{
  "term_id": "UNKNOWN:0001",
  "gene_symbol": "NDRG2",
  "term_label": "Unknown molecular function",
  "gene_name": "Protein NDRG2",
  "gene": "UniProtKB:Q9UN36"
}